{
  "gene": "UniProtKB:Q9HBE1",
  "gene_name": "POZ-, AT hook-, and zinc finger-containing protein 1",
  "gene_symbol": "PATZ1",
  "term_id": "GO:0000978",
  "term_label": "RNA polymerase II cis-regulatory region sequence-specific DNA binding"
}